{
  "term_id": "GO:0006491",
  "gene_symbol": "ST8SIA3",
  "gene_name": "Sia-alpha-2,3-Gal-beta-1,4-GlcNAc-R:alpha 2,8-sialyltransferase",
  "term_label": "N-glycan processing",
  "gene": "UniProtKB:O43173"
}